L-arabitol catabolic process [GO:0051158] (biological process) Definition: The chemical reactions and pathways resulting in the breakdown of L-arabitol, the pentitol derived from arabinose or lyxose by reduction of the aldehyde group. Sources: ISBN:0198506732 Also known as: L-arabitol breakdown, L-arabitol catabolism, L-arabitol degradation Relationships: is_a arabitol catabolic process [GO:0051157] Subtypes: GO:0019590